{
  "term_id": "UNKNOWN:0001",
  "term_label": "Unknown molecular function",
  "gene_symbol": "FAM236B",
  "gene": "UniProtKB:A0A1B0GV22",
  "gene_name": "Protein FAM236B"
}